{
  "gene": "UniProtKB:Q9P1Z0",
  "gene_symbol": "ZBTB4",
  "term_id": "GO:0000981",
  "gene_name": "Zinc finger and BTB domain-containing protein 4",
  "term_label": "DNA-binding transcription factor activity, RNA polymerase II-specific"
}